{
  "term_id": "GO:0071880",
  "gene": "UniProtKB:P25100",
  "gene_symbol": "ADRA1D",
  "gene_name": "Alpha-1D adrenergic receptor",
  "term_label": "adenylate cyclase-activating adrenergic receptor signaling pathway"
}